{
  "gene_name": "Killer cell immunoglobulin-like receptor, three Ig domains pseudogene 1",
  "gene_symbol": "KIR3DP1",
  "gene": "UniProtKB:A0A0G2JN01",
  "term_id": "GO:0002767",
  "term_label": "immune response-inhibiting cell surface receptor signaling pathway"
}